{
  "term_id": "GO:0003730",
  "gene_name": "Deleted in azoospermia-like",
  "gene_symbol": "DAZL",
  "gene": "UniProtKB:Q92904",
  "term_label": "mRNA 3'-UTR binding"
}